{
  "term_id": "GO:0005737",
  "term_label": "cytoplasm",
  "gene": "UniProtKB:P12268",
  "gene_name": "Inosine-5'-monophosphate dehydrogenase 2",
  "gene_symbol": "IMPDH2"
}